{
  "gene_name": "Centromere protein T",
  "term_label": "chromosome segregation",
  "gene": "UniProtKB:Q96BT3",
  "term_id": "GO:0007059",
  "gene_symbol": "CENPT"
}